{
  "term_id": "GO:0006275",
  "term_label": "regulation of DNA replication",
  "gene": "UniProtKB:Q7Z6E9",
  "gene_name": "E3 ubiquitin-protein ligase RBBP6",
  "gene_symbol": "RBBP6"
}